regulation of response to biotic stimulus [GO:0002831] (biological process) Relationships: is a type of GO:0048583; regulates response to biotic stimulus [GO:0009607] Subtypes: regulation of antimicrobial humoral response [GO:0002759], negative regulation of response to biotic stimulus [GO:0002832], GO:0002833, regulation of response to tumor cell [GO:0002834], regulation of systemic acquired resistance [GO:0010112], GO:0031664, regulation of innate immune response [GO:0045088], regulation of defense response to virus [GO:0050688], regulation of neutrophil mediated killing of symbiont cell [GO:0070949], regulation of defense response to fungus [GO:1900150], regulation of defense response to bacterium [GO:1900424], regulation of filamentous growth of a population of unicellular organisms in response to biotic stimulus [GO:1900443], regulation of response to cell cycle checkpoint signaling [GO:1902145], regulation of defense response to oomycetes [GO:1902288], regulation of xenophagy [GO:1904415], GO:2000068 Definition: Any process that modulates the frequency, rate, or extent of a response to biotic stimulus. Note: Note that this term is in the subset of terms that should not be used for direct gene product annotation. Instead, select a child term or, if no appropriate child term exists, please request a new term. Direct annotations to this term may be amended during annotation QC. Sources: GOC:add